{
  "gene_name": "Small nuclear ribonucleoprotein E",
  "gene": "UniProtKB:P62304",
  "term_label": "spliceosomal snRNP assembly",
  "gene_symbol": "SNRPE",
  "term_id": "GO:0000387"
}